{
  "term_label": "deSUMOylase activity",
  "gene": "UniProtKB:Q9P0U3",
  "gene_symbol": "SENP1",
  "gene_name": "Sentrin-specific protease 1",
  "term_id": "GO:0016929"
}